{
  "gene_name": "Carotenoid-cleaving dioxygenase, mitochondrial",
  "gene_symbol": "BCO2",
  "gene": "UniProtKB:Q9BYV7",
  "term_label": "retinal metabolic process",
  "term_id": "GO:0042574"
}